structural constituent of ribosome [GO:0003735] (molecular function) Relationships: is a type of structural molecule activity [GO:0005198]; occurs in ribosome [GO:0005840] Definition: The action of a molecule that contributes to the structural integrity of the ribosome. Also known as: ribosomal protein, ribosomal RNA Sources: GOC:mah Note: Note that this term may be used to annotate ribosomal RNAs as well as ribosomal proteins.